{
  "term_id": "GO:0033147",
  "gene": "UniProtKB:Q63ZY3",
  "term_label": "negative regulation of intracellular estrogen receptor signaling pathway",
  "gene_name": "KN motif and ankyrin repeat domain-containing protein 2",
  "gene_symbol": "KANK2"
}